Rab-protein geranylgeranyltransferase complex [GO:0005968] (cellular component) Relationships: is a type of transferase complex [GO:1990234]; is part of cytoplasm [GO:0005737] Also known as: GGTase-II complex, Rab geranylgeranyltransferase complex, RabGGTase complex Definition: An protein-containing complex which catalyzes of the transfer of a geranyl-geranyl group from geranylgeranyl pyrophosphate to a Rab protein. In mammals it is composed of an alpha and a beta subunit, and associates with an accessory protein Rep (Rab escort protein). References: PMID:11886217 Sources: GOC:jl